protein localization to nucleoplasm [GO:1990173] (biological process) Subtypes: GO:1903405 Relationships: is a type of protein localization to nucleus [GO:0034504] Definition: A process in which a protein is transported to, or maintained in, a location within the nucleoplasm. Also known as: protein localisation to nucleoplasm, nucleolus to nucleoplasm transport References: PMID:22918952 Sources: GOC:mah